glycinergic synapse [GO:0098690] (cellular component) Definition: A synapse that uses glycine as a neurotransmitter. Sources: GOC:dos Relationships: is a type of synapse [GO:0045202]